positive regulation of interleukin-21 production [GO:0032745] (biological process) Relationships: is a type of positive regulation of cytokine production [GO:0001819]; is a type of regulation of interleukin-21 production [GO:0032665]; positively regulates interleukin-21 production [GO:0032625] Definition: Any process that activates or increases the frequency, rate, or extent of interleukin-21 production. Also known as: positive regulation of IL-21 production, up regulation of interleukin-21 production, up-regulation of interleukin-21 production, upregulation of interleukin-21 production, activation of interleukin-21 production, positive regulation of interleukin-21 biosynthetic process, stimulation of interleukin-21 production Sources: GOC:mah